{
  "term_label": "death-inducing signaling complex",
  "gene": "UniProtKB:P42574",
  "term_id": "GO:0031264",
  "gene_name": "Caspase-3",
  "gene_symbol": "CASP3"
}